symbiont-mediated evasion of DNA end degradation by host [GO:0099016] (biological process) References: PMID:11894948, PMID:16949369 Sources: GOC:dos, VZ:3963 Also known as: DNA end degradation evasion by virus, evasion of DNA end degradation by host, evasion by virus of DNA end degradation Definition: A process by which a symbiont evades and ends degradation of its DNA when free DNA ends are exposed. DNA ends are exposed during the life cycle of some viruses and these are targeted by host cells to destroy the virus. For example, some bacteriophages encode proteins that bind to free viral DNA ends, protecting them from degradation by host exonucleases. Relationships: is a type of GO:0141177